{
  "gene_symbol": "AEBP1",
  "gene_name": "Adipocyte enhancer-binding protein 1",
  "term_label": "regulation of DNA-templated transcription",
  "gene": "UniProtKB:Q8IUX7",
  "term_id": "GO:0006355"
}